stereocilium membrane [GO:0060171] (cellular component) Definition: The portion of the plasma membrane surrounding a stereocilium. Sources: GOC:dph, GOC:rph Relationships: is a type of neuron projection membrane [GO:0032589]; is part of intracellular anatomical structure [GO:0005622]; is part of stereocilium [GO:0032420]